positive regulation of mast cell differentiation [GO:0060376] (biological process) Sources: GOC:dph, GOC:tb Relationships: is a type of positive regulation of myeloid leukocyte differentiation [GO:0002763]; is a type of regulation of mast cell differentiation [GO:0060375]; positively regulates mast cell differentiation [GO:0060374] Definition: Any process that increases the rate, frequency or extent of mast cell differentiation, the process in which a relatively unspecialized myeloid precursor cell acquires the specialized features of a mast cell. A mast cell is a cell that is found in almost all tissues containing numerous basophilic granules and capable of releasing large amounts of histamine and heparin upon activation.